{
  "gene_symbol": "TMED8",
  "gene": "UniProtKB:Q6PL24",
  "gene_name": "Protein TMED8",
  "term_label": "Unknown biological process",
  "term_id": "UNKNOWN:0002"
}